mononuclear cell migration [GO:0071674] (biological process) Relationships: is a type of leukocyte migration [GO:0050900] Subtypes: monocyte chemotaxis [GO:0002548], monocyte extravasation [GO:0035696], monocyte migration into blood stream [GO:0035703], dendritic cell migration [GO:0036336], lymphocyte migration [GO:0072676], macrophage migration [GO:1905517] Sources: GOC:mah Definition: The movement of a mononuclear cell within or between different tissues and organs of the body. Regulation: regulated by regulation of mononuclear cell migration [GO:0071675]; negatively regulated by negative regulation of mononuclear cell migration [GO:0071676]; positively regulated by positive regulation of mononuclear cell migration [GO:0071677]